{
  "term_label": "GTPase activity",
  "gene_name": "Ras-related protein Rab-1A",
  "term_id": "GO:0003924",
  "gene_symbol": "RAB1A",
  "gene": "UniProtKB:P62820"
}